phasic smooth muscle contraction [GO:0014821] (biological process) Sources: GOC:mtg_muscle Definition: A process in which force is generated within phasic smooth muscle tissue, resulting in a change in muscle geometry. Force generation involves a chemo-mechanical energy conversion step that is carried out by the actin/myosin complex activity, which generates force through ATP hydrolysis. In the phasic smooth muscle, the muscle contraction occurs without an ordered sarcomeric structure. Phasic smooth muscle contraction occurs in a series of discrete contractions and relaxations. Subtypes: vein smooth muscle contraction [GO:0014826], intestine smooth muscle contraction [GO:0014827], distal stomach smooth muscle contraction [GO:0014828], ureter smooth muscle contraction [GO:0014849], peristalsis [GO:0030432] Relationships: is a type of GO:0006939